{
  "gene_symbol": "CKLF",
  "gene_name": "Chemokine-like factor",
  "term_id": "UNKNOWN:0002",
  "gene": "UniProtKB:Q9UBR5",
  "term_label": "Unknown biological process"
}